RNA polymerase II CTD heptapeptide repeat Y1 kinase activity [GO:0140833] (molecular function) Relationships: is_a RNA polymerase II CTD heptapeptide repeat kinase activity [GO:0008353] Definition: Catalysis of the reaction: ATP + RNA polymerase II large subunit CTD heptapeptide repeat (consensus YSPTSPS) = ADP + H+ + RNA polymerase II large subunit phosphotyrosine (position 1). References: PMID:28248323 Also known as: RNA polymerase II C-terminal domain Y1 kinase activity